{
  "gene": "UniProtKB:P0DOY2",
  "gene_name": "Immunoglobulin lambda constant 2",
  "gene_symbol": "IGLC2",
  "term_label": "immunoglobulin mediated immune response",
  "term_id": "GO:0016064"
}